tRNA pseudouridine(13) synthase activity [GO:0160150] (molecular function) Relationships: is a type of tRNA pseudouridine synthase activity [GO:0106029] Definition: Catalysis of the reaction: uridine(13) in tRNA = pseudouridine(13) in tRNA. Sources: EC:5.4.99.27